{
  "term_id": "UNKNOWN:0003",
  "gene_symbol": "LINC00472",
  "term_label": "Unknown cellular component",
  "gene": "UniProtKB:Q9H8W2",
  "gene_name": "Putative uncharacterized protein encoded by LINC00472"
}